{
  "gene_symbol": "TBRG4",
  "term_label": "regulation of mitochondrial mRNA stability",
  "gene": "UniProtKB:Q969Z0",
  "term_id": "GO:0044528",
  "gene_name": "FAST kinase domain-containing protein 4"
}